telencephalon cell migration [GO:0022029] (biological process) Definition: The orderly movement of a cell from one site to another at least one of which is located in the telencephalon. Relationships: is a type of forebrain cell migration [GO:0021885]; is part of telencephalon development [GO:0021537] Subtypes: cerebral cortex cell migration [GO:0021795], substrate-independent telencephalic tangential migration [GO:0021826], subpallium cell migration [GO:0021980], tangential migration from the subventricular zone to the olfactory bulb [GO:0022028], telencephalon glial cell migration [GO:0022030] Sources: GOC:cls, GOC:curators, GOC:dgh, GOC:dph, GOC:jid